photoreceptor outer segment membrane [GO:0042622] (cellular component) Sources: GOC:jl Relationships: is a type of ciliary membrane [GO:0060170]; is part of photoreceptor outer segment [GO:0001750] Definition: The membrane surrounding the outer segment of a vertebrate photoreceptor.